neutrophil mediated cytotoxicity [GO:0070942] (biological process) Regulation: regulated by regulation of neutrophil mediated cytotoxicity [GO:0070948]; negatively regulated by negative regulation of neutrophil mediated cytotoxicity [GO:0070954]; positively regulated by positive regulation of neutrophil mediated cytotoxicity [GO:0070960] Subtypes: neutrophil-mediated killing of symbiont cell [GO:0070943] Relationships: is a type of leukocyte mediated cytotoxicity [GO:0001909]; is a type of GO:0002446 Definition: The directed killing of a target cell by a neutrophil. Also known as: neutrophil mediated cell killing Sources: GOC:add, ISBN:0781765196